{
  "term_label": "octopamine biosynthetic process",
  "gene": "UniProtKB:Q6UVY6",
  "gene_symbol": "MOXD1",
  "term_id": "GO:0006589",
  "gene_name": "DBH-like monooxygenase protein 1"
}